{
  "gene": "UniProtKB:Q8N907",
  "term_id": "GO:0016015",
  "gene_symbol": "DAND5",
  "term_label": "morphogen activity",
  "gene_name": "DAN domain family member 5"
}